{
  "term_label": "Unknown molecular function",
  "term_id": "UNKNOWN:0001",
  "gene_name": "Contactin associated protein family member 3C (Fragment)",
  "gene": "UniProtKB:A0A1B0GTE1",
  "gene_symbol": "CNTNAP3C"
}